G protein-coupled receptor signaling pathway coupled to cGMP nucleotide second messenger [GO:0007199] (biological process) Sources: GOC:mah, GOC:signaling, ISBN:0815316194 Definition: The series of molecular signals generated as a consequence of a G protein-coupled receptor binding to its physiological ligand, followed by activation of guanylyl cyclase (GC) activity and a subsequent increase in the concentration of cyclic GMP (cGMP). Also known as: G protein signaling, coupled to cGMP nucleotide second messenger, G protein signalling, coupled to cGMP nucleotide second messenger, G-protein coupled receptor signaling pathway coupled to cGMP nucleotide second messenger, G-protein signaling, coupled to cGMP nucleotide second messenger, G-protein signalling, coupled to cGMP nucleotide second messenger, GPCR signaling pathway via activation of guanylate cyclase activity, GPCR signaling pathway via cGMP second messenger, guanylate cyclase-activating G-protein coupled receptor signaling pathway Relationships: is a type of G protein-coupled receptor signaling pathway, coupled to cyclic nucleotide second messenger [GO:0007187]